aerobic raffinose catabolic process [GO:0036259] (biological process) Definition: The chemical reactions and pathways resulting in the breakdown of raffinose that occur in the presence of oxygen. References: PMID:10082789 Sources: GOC:al Also known as: aerobic raffinose breakdown, aerobic raffinose catabolism, aerobic raffinose degradation Relationships: is a type of raffinose catabolic process [GO:0034484]